{
  "term_id": "UNKNOWN:0001",
  "gene_name": "T cell receptor beta variable 5-6",
  "term_label": "Unknown molecular function",
  "gene": "UniProtKB:A0A599",
  "gene_symbol": "TRBV5-6"
}